negative regulation of toll-like receptor 7 signaling pathway [GO:0034156] (biological process) Definition: Any process that stops, prevents, or reduces the frequency, rate, or extent of toll-like receptor 7 signaling pathway. References: PMID:16551253, PMID:17328678 Sources: GOC:add Also known as: negative regulation of TLR7 signaling pathway, negative regulation of toll-like receptor 7 signalling pathway Relationships: is_a regulation of toll-like receptor 7 signaling pathway [GO:0034155]; is a type of negative regulation of cytoplasmic pattern recognition receptor signaling pathway [GO:0039532]; negatively regulates toll-like receptor 7 signaling pathway [GO:0034154]